{
  "gene_symbol": "FASTKD3",
  "gene_name": "FAST kinase domain-containing protein 3, mitochondrial",
  "gene": "UniProtKB:Q14CZ7",
  "term_id": "GO:0035770",
  "term_label": "ribonucleoprotein granule"
}